{
  "gene_name": "Leukemia-associated protein 7",
  "gene": "UniProtKB:Q6UYE1",
  "term_id": "UNKNOWN:0003",
  "gene_symbol": "DLEU7",
  "term_label": "Unknown cellular component"
}